positive regulation of bone mineralization [GO:0030501] (biological process) Relationships: is a type of regulation of bone mineralization [GO:0030500]; is a type of positive regulation of ossification [GO:0045778]; is a type of positive regulation of biomineral tissue development [GO:0070169]; positively regulates GO:0030282 Definition: Any process that activates or increases the frequency, rate or extent of bone mineralization. Also known as: up regulation of bone mineralization, up-regulation of bone mineralization, upregulation of bone mineralization, activation of bone mineralization, stimulation of bone mineralization Subtypes: positive regulation of bone mineralization involved in bone maturation [GO:1900159] Sources: GOC:go_curators